{
  "gene": "UniProtKB:Q01344",
  "term_id": "GO:0009897",
  "term_label": "external side of plasma membrane",
  "gene_symbol": "IL5RA",
  "gene_name": "Interleukin-5 receptor subunit alpha"
}